{
  "gene_symbol": "RBBP4",
  "term_label": "histone binding",
  "gene": "UniProtKB:Q09028",
  "term_id": "GO:0042393",
  "gene_name": "Histone-binding protein RBBP4"
}